{
  "gene_symbol": "PFKFB1",
  "term_label": "6-phosphofructo-2-kinase activity",
  "gene": "UniProtKB:P16118",
  "term_id": "GO:0003873",
  "gene_name": "6-phosphofructo-2-kinase_fructose-2,6-bisphosphatase 1"
}